phospholipid catabolic process [GO:0009395] (BP) Sources: ISBN:0198506732 Regulation: regulated by GO:0060696; positively regulated by positive regulation of phospholipid catabolic process [GO:0060697] Also known as: phospholipid breakdown, phospholipid catabolism, phospholipid degradation Subtypes: sphingomyelin catabolic process [GO:0006685], GO:0045339, glycerophospholipid catabolic process [GO:0046475], GO:0051874, 5alpha,9alpha,10beta-labda-8(20),13-dien-15-yl diphosphate catabolic process [GO:1901948], GO:1902242, geranylgeranyl diphosphate catabolic process [GO:1902247], ceramide phosphoethanolamine catabolic process [GO:1905372] Definition: The chemical reactions and pathways resulting in the breakdown of phospholipids, any lipid containing phosphoric acid as a mono- or diester. Relationships: is a type of phospholipid metabolic process [GO:0006644]; is a type of GO:0016042; is a type of organophosphate catabolic process [GO:0046434]